{
  "gene_name": "SUMO-interacting motif-containing protein 1",
  "gene_symbol": "SIMC1",
  "term_label": "Unknown cellular component",
  "gene": "UniProtKB:Q8NDZ2",
  "term_id": "UNKNOWN:0003"
}